larval wandering behavior [GO:0035180] (biological process) Definition: The movement of a third instar larva through a substrate in search of a pupation site. This movement occurs without feeding and is characterized by short bursts of forward movement, separated by stops and repeated side-to-side head probes, followed normally by a change in direction. Relationships: is a type of larval locomotory behavior [GO:0008345] References: PMID:12848927, PMID:12956960 Also known as: larval wandering behaviour